{
  "gene": "UniProtKB:Q8TF27",
  "term_id": "UNKNOWN:0002",
  "term_label": "Unknown biological process",
  "gene_symbol": "AGAP11",
  "gene_name": "Arf-GAP with GTPase, ANK repeat and PH domain-containing protein 11"
}